{
  "gene": "UniProtKB:Q5TIA1",
  "gene_symbol": "MEI1",
  "term_label": "Unknown molecular function",
  "gene_name": "Meiosis inhibitor protein 1",
  "term_id": "UNKNOWN:0001"
}